lactate transmembrane transporter activity [GO:0015129] (molecular function) Relationships: is a type of GO:0008028; is part of lactate transmembrane transport [GO:0035873] Subtypes: lactate:proton symporter activity [GO:0015650] Definition: Enables the transfer of lactate from one side of a membrane to the other. Lactate is 2-hydroxypropanoate, CH3-CHOH-COOH; L(+)-lactate is formed by anaerobic glycolysis in animal tissues, and DL-lactate is found in sour milk, molasses and certain fruit juices. Also known as: monocarboxylate (lactate, pyruvate, mevalonate) uptake/efflux porter activity Sources: GOC:ai, ISBN:0198506732